{
  "gene_name": "Refilin-A",
  "term_label": "actin filament bundle organization",
  "gene": "UniProtKB:Q6ZTI6",
  "term_id": "GO:0061572",
  "gene_symbol": "RFLNA"
}